{
  "term_label": "protein O-linked glycosylation via mannose",
  "term_id": "GO:0035269",
  "gene": "UniProtKB:Q9UKY4",
  "gene_symbol": "POMT2",
  "gene_name": "Protein O-mannosyl-transferase 2"
}